{
  "gene_name": "Zinc finger matrin-type protein 3",
  "term_id": "UNKNOWN:0001",
  "gene": "UniProtKB:Q9HA38",
  "gene_symbol": "ZMAT3",
  "term_label": "Unknown molecular function"
}